{
  "term_id": "GO:0010818",
  "term_label": "T cell chemotaxis",
  "gene_symbol": "CXCL16",
  "gene_name": "C-X-C motif chemokine 16",
  "gene": "UniProtKB:Q9H2A7"
}